{
  "gene_symbol": "AGBL4",
  "gene_name": "Cytosolic carboxypeptidase 6",
  "gene": "UniProtKB:Q5VU57",
  "term_id": "UNKNOWN:0002",
  "term_label": "Unknown biological process"
}